{
  "term_id": "UNKNOWN:0002",
  "gene_symbol": "STYK1",
  "gene_name": "Tyrosine-protein kinase STYK1",
  "gene": "UniProtKB:Q6J9G0",
  "term_label": "Unknown biological process"
}